{
  "gene_symbol": "DBX2",
  "gene_name": "Homeobox protein DBX2",
  "term_id": "UNKNOWN:0003",
  "term_label": "Unknown cellular component",
  "gene": "UniProtKB:Q6ZNG2"
}